{
  "gene_name": "Nuclear factor erythroid 2-related factor 3",
  "term_id": "GO:0000978",
  "term_label": "RNA polymerase II cis-regulatory region sequence-specific DNA binding",
  "gene_symbol": "NFE2L3",
  "gene": "UniProtKB:Q9Y4A8"
}